{
  "gene": "UniProtKB:Q9NZJ9",
  "term_id": "GO:0034432",
  "gene_symbol": "NUDT4",
  "gene_name": "Diphosphoinositol polyphosphate phosphohydrolase 2",
  "term_label": "bis(5'-adenosyl)-pentaphosphatase activity"
}